{
  "gene": "UniProtKB:O43299",
  "gene_symbol": "AP5Z1",
  "term_id": "UNKNOWN:0002",
  "term_label": "Unknown biological process",
  "gene_name": "AP-5 complex subunit zeta-1"
}